{
  "term_id": "GO:0043065",
  "gene_name": "Dual specificity protein phosphatase 6",
  "gene": "UniProtKB:Q16828",
  "term_label": "positive regulation of apoptotic process",
  "gene_symbol": "DUSP6"
}